positive regulation of TORC2 signaling [GO:1904515] (biological process) Also known as: positive regulation of TORC2 signal transduction, up regulation of TORC2 signal transduction, up regulation of TORC2 signaling, up-regulation of TORC2 signal transduction, up-regulation of TORC2 signaling, upregulation of TORC2 signal transduction, upregulation of TORC2 signaling, activation of TORC2 signal transduction, activation of TORC2 signaling Relationships: is a type of positive regulation of TOR signaling [GO:0032008]; is a type of regulation of TORC2 signaling [GO:1903939]; RO_0002213 TORC2 signaling [GO:0038203] Definition: Any process that activates or increases the frequency, rate or extent of TORC2 signaling. References: PMID:25590601 Sources: GOC:TermGenie, GO_REF:0000058